{
  "term_label": "biliverdin reductase [NAD(P)H] activity",
  "gene": "UniProtKB:P53004",
  "gene_symbol": "BLVRA",
  "gene_name": "Biliverdin reductase A",
  "term_id": "GO:0004074"
}